{
  "term_label": "cilium assembly",
  "term_id": "GO:0060271",
  "gene_symbol": "DCDC2",
  "gene": "UniProtKB:Q9UHG0",
  "gene_name": "Doublecortin domain-containing protein 2"
}